{
  "gene_name": "Calcium_calmodulin-dependent protein kinase type 1D",
  "term_id": "GO:0071622",
  "gene_symbol": "CAMK1D",
  "term_label": "regulation of granulocyte chemotaxis",
  "gene": "UniProtKB:Q8IU85"
}